{
  "term_id": "UNKNOWN:0003",
  "gene_symbol": "CYP4A11",
  "term_label": "Unknown cellular component",
  "gene_name": "Cytochrome P450 4A11",
  "gene": "UniProtKB:Q02928"
}